regulation of shelterin complex assembly [GO:1904790] (biological process) Also known as: regulation of Pot1 complex assembly, regulation of Pot1-Tpz1 complex assembly, regulation of shelterin complex formation, regulation of telosome assembly References: PMID:24270157 Sources: GOC:BHF, GOC:BHF_telomere, GOC:TermGenie, GOC:nc, GO_REF:0000058 Subtypes: negative regulation of shelterin complex assembly [GO:1904791], positive regulation of shelterin complex assembly [GO:1904792] Definition: Any process that modulates the frequency, rate or extent of shelterin complex assembly. Relationships: is a type of regulation of protein-containing complex assembly [GO:0043254]; regulates shelterin complex assembly [GO:0071573]